{
  "gene_symbol": "IL6R",
  "gene_name": "Interleukin-6 receptor subunit alpha",
  "gene": "UniProtKB:P08887",
  "term_id": "GO:0009897",
  "term_label": "external side of plasma membrane"
}